{
  "term_id": "UNKNOWN:0001",
  "gene_symbol": "CLPTM1",
  "gene_name": "Putative lipid scramblase CLPTM1",
  "gene": "UniProtKB:O96005",
  "term_label": "Unknown molecular function"
}